{
  "gene_symbol": "SLC1A7",
  "term_id": "GO:0005886",
  "gene": "UniProtKB:O00341",
  "gene_name": "Excitatory amino acid transporter 5",
  "term_label": "plasma membrane"
}